2'-deoxyadenosine deaminase activity [GO:0046936] (molecular function) Definition: Catalysis of the reaction: 2'-deoxyadenosine + H+ + H2O = 2'-deoxyinosine + NH4+. Sources: GOC:ai, RHEA:28190 Relationships: is a type of hydrolase activity, acting on carbon-nitrogen (but not peptide) bonds, in cyclic amidines [GO:0016814]; is a type of deaminase activity [GO:0019239] Also known as: deoxyadenosine deaminase reaction